{
  "term_label": "immunoglobulin complex",
  "gene": "UniProtKB:A0A075B6I3",
  "gene_name": "Probable non-functional immunoglobulin lambda variable 11-55",
  "term_id": "GO:0019814",
  "gene_symbol": "IGLV11-55"
}